{
  "gene": "UniProtKB:Q13822",
  "term_label": "phosphatidylcholine lysophospholipase activity",
  "term_id": "GO:0004622",
  "gene_symbol": "ENPP2",
  "gene_name": "Ectonucleotide pyrophosphatase_phosphodiesterase family member 2"
}